morphogenesis of an endothelium [GO:0003159] (biological process) Subtypes: endothelial tube morphogenesis [GO:0061154] Definition: The process in which the anatomical structure of an endothelium is generated and organized. Endothelium refers to the layer of cells lining blood vessels, lymphatics, the heart, and serous cavities, and is derived from bone marrow or mesoderm. Corneal endothelium is a special case, derived from neural crest cells. Sources: GOC:mtg_heart Relationships: is a type of morphogenesis of an epithelium [GO:0002009]; is part of GO:0003158